{
  "gene_symbol": "DYRK4",
  "term_id": "UNKNOWN:0002",
  "gene_name": "Dual specificity tyrosine-phosphorylation-regulated kinase 4",
  "term_label": "Unknown biological process",
  "gene": "UniProtKB:Q9NR20"
}